{
  "gene": "UniProtKB:O95876",
  "term_id": "GO:0044782",
  "gene_symbol": "WDPCP",
  "gene_name": "WD repeat-containing and planar cell polarity effector protein fritz homolog",
  "term_label": "cilium organization"
}